cellular response to far red light [GO:0071490] (BP) Also known as: cellular response to far red light stimulus Definition: Any process that results in a change in state or activity of a cell (in terms of movement, secretion, enzyme production, gene expression, etc.) as a result of far red light stimulus. Far red light is electromagnetic radiation of wavelength 700-800nm. An example of this response is seen at the beginning of many plant species developmental stages. These include germination, and the point when cotyledon expansion is triggered. In certain species these processes take place in response to absorption of red light by the pigment molecule phytochrome, but the signal can be reversed by exposure to far red light. During the initial phase the phytochrome molecule is only present in the red light absorbing form, but on absorption of red light it changes to a far red light absorbing form, triggering progress through development. An immediate short period of exposure to far red light entirely returns the pigment to its initial state and prevents triggering of the developmental process. A thirty minute break between red and subsequent far red light exposure renders the red light effect irreversible, and development then occurs regardless of whether far red light exposure subsequently occurs. Subtypes: far-red light signaling pathway [GO:0010018] Sources: GOC:mah Relationships: is a type of response to far red light [GO:0010218]; is a type of GO:0071489